vesicle docking involved in exocytosis [GO:0006904] (BP) Definition: The initial attachment of a vesicle membrane to a target membrane, mediated by proteins protruding from the membrane of the vesicle and the target membrane, that contributes to exocytosis. Also known as: vesicle docking during exocytosis References: PMID:22438915 Sources: GOC:aruk, GOC:bc, GOC:jid Relationships: is a type of vesicle docking [GO:0048278]; is a type of exocytic process [GO:0140029] Subtypes: synaptic vesicle docking [GO:0016081], dense core granule docking [GO:0061790], exocytic insertion of neurotransmitter receptor to plasma membrane [GO:0098881]